{
  "gene_name": "Indolethylamine N-methyltransferase",
  "gene": "UniProtKB:O95050",
  "term_id": "GO:0005829",
  "term_label": "cytosol",
  "gene_symbol": "INMT"
}